{
  "term_label": "structural constituent of ribosome",
  "gene": "UniProtKB:Q92901",
  "gene_name": "Ribosomal protein uL3-like",
  "term_id": "GO:0003735",
  "gene_symbol": "RPL3L"
}